{
  "gene": "UniProtKB:Q8N8R3",
  "term_id": "GO:0005739",
  "gene_symbol": "SLC25A29",
  "gene_name": "Mitochondrial basic amino acids transporter",
  "term_label": "mitochondrion"
}